cellular response to singlet oxygen [GO:0071452] (biological process) Relationships: is a type of response to singlet oxygen [GO:0000304]; is a type of cellular response to reactive oxygen species [GO:0034614] Sources: GOC:mah Definition: Any process that results in a change in state or activity of a cell (in terms of movement, secretion, enzyme production, gene expression, etc.) as a result of a singlet oxygen stimulus. Singlet oxygen is a dioxygen (O2) molecule in which two 2p electrons have similar spin. Singlet oxygen is more highly reactive than the form in which these electrons are of opposite spin, and it is produced in mutant chloroplasts lacking carotenoids and by leukocytes during metabolic burst.